lung morphogenesis [GO:0060425] (biological process) Relationships: is a type of GO:0009887; is part of lung development [GO:0030324] Definition: The process in which the anatomical structures of the lung are generated and organized. Subtypes: left lung morphogenesis [GO:0060460], right lung morphogenesis [GO:0060461] Sources: GOC:dph